amino acid import [GO:0043090] (biological process) Definition: The directed movement of amino acids into a cell or organelle. Also known as: amino acid uptake Relationships: is a type of amino acid transport [GO:0006865] Sources: GOC:jl